creatinine catabolic process [GO:0006602] (biological process) Subtypes: creatinine catabolic process to formate [GO:0019621] Also known as: creatinine breakdown, creatinine catabolism, creatinine degradation Relationships: is a type of creatinine metabolic process [GO:0046449]; is a type of GO:0072340 Definition: The chemical reactions and pathways resulting in the breakdown of creatinine, 2-amino-1,5-dihydro-1-methyl-4H-imidazol-4-one, an end product of creatine metabolism and a normal constituent of urine. Sources: ISBN:0198506732